myosin II complex [GO:0016460] (cellular component) Subtypes: muscle myosin complex [GO:0005859] Definition: A myosin complex containing two class II myosin heavy chains, two myosin essential light chains and two myosin regulatory light chains. Also known as classical myosin or conventional myosin, the myosin II class includes the major muscle myosin of vertebrate and invertebrate muscle, and is characterized by alpha-helical coiled coil tails that self assemble to form a variety of filament structures. Sources: Wikipedia:Myosin Relationships: is a type of myosin complex [GO:0016459] Also known as: conventional myosin